{
  "term_id": "GO:0031643",
  "term_label": "positive regulation of myelination",
  "gene": "UniProtKB:Q8N5U6",
  "gene_name": "E3 ubiquitin-protein ligase RNF10",
  "gene_symbol": "RNF10"
}